defasciculation of motor neuron axon [GO:0007415] (biological process) Definition: Separation of a motor axon away from a bundle of axons known as a fascicle. Sources: GOC:dgh Relationships: is a type of GO:0007414